positive regulation of mitotic centrosome separation [GO:0046604] (biological process) Sources: GOC:ai Also known as: up regulation of mitotic centrosome separation, up-regulation of mitotic centrosome separation, upregulation of mitotic centrosome separation, activation of mitotic centrosome separation, stimulation of mitotic centrosome separation Definition: Any process that activates or increases the frequency, rate or extent of centrosome separation. Relationships: is a type of regulation of mitotic centrosome separation [GO:0046602]; is a type of positive regulation of cell cycle process [GO:0090068]; positively regulates mitotic centrosome separation [GO:0007100]